{
  "gene_symbol": "LOC124905412",
  "gene_name": "Homeobox domain-containing protein",
  "gene": "UniProtKB:A0A1B0GW55",
  "term_id": "GO:0000981",
  "term_label": "DNA-binding transcription factor activity, RNA polymerase II-specific"
}